{
  "term_id": "GO:0006508",
  "gene_symbol": "FAP",
  "gene_name": "Prolyl endopeptidase FAP",
  "gene": "UniProtKB:Q12884",
  "term_label": "proteolysis"
}